{
  "term_label": "glycine cleavage complex",
  "gene_symbol": "GCSH",
  "gene_name": "Glycine cleavage system H protein, mitochondrial",
  "term_id": "GO:0005960",
  "gene": "UniProtKB:P23434"
}